{
  "gene_symbol": "AR",
  "term_label": "androgen receptor signaling pathway",
  "gene_name": "Androgen receptor",
  "term_id": "GO:0030521",
  "gene": "UniProtKB:P10275"
}